{
  "term_id": "UNKNOWN:0003",
  "gene": "UniProtKB:Q8NDV1",
  "term_label": "Unknown cellular component",
  "gene_name": "Alpha-N-acetylgalactosaminide alpha-2,6-sialyltransferase 3",
  "gene_symbol": "ST6GALNAC3"
}